{
  "gene_name": "Zinc finger imprinted 3",
  "gene_symbol": "ZIM3",
  "term_label": "regulation of transcription by RNA polymerase II",
  "gene": "UniProtKB:Q96PE6",
  "term_id": "GO:0006357"
}